{
  "term_label": "regulation of DNA-templated transcription",
  "gene_name": "Vasculin",
  "term_id": "GO:0006355",
  "gene_symbol": "GPBP1",
  "gene": "UniProtKB:Q86WP2"
}